{
  "gene": "UniProtKB:Q13546",
  "gene_name": "Receptor-interacting serine_threonine-protein kinase 1",
  "term_id": "GO:0005737",
  "term_label": "cytoplasm",
  "gene_symbol": "RIPK1"
}